regulation of DNA endoreduplication [GO:0032875] (BP) Also known as: regulation of DNA endoreplication, regulation of DNA re-duplication Definition: Any process that modulates the frequency, rate or extent of DNA endoreduplication. Sources: GOC:mah Subtypes: negative regulation of DNA endoreduplication [GO:0032876], GO:0032877 Relationships: is a type of GO:0010564; is a type of regulation of DNA-templated DNA replication [GO:0090329]; regulates DNA endoreduplication [GO:0042023]